{
  "term_label": "Unknown molecular function",
  "gene_name": "Uncharacterized protein C17orf80",
  "term_id": "UNKNOWN:0001",
  "gene": "UniProtKB:Q9BSJ5",
  "gene_symbol": "C17orf80"
}